{
  "term_label": "plasma membrane",
  "gene_symbol": "ENOX1",
  "gene_name": "Ecto-NOX disulfide-thiol exchanger 1",
  "term_id": "GO:0005886",
  "gene": "UniProtKB:Q8TC92"
}